{
  "term_id": "GO:0042476",
  "gene": "UniProtKB:Q6PRD7",
  "term_label": "odontogenesis",
  "gene_symbol": "CEMP1",
  "gene_name": "Cementoblastoma-derived protein 1"
}